positive regulation of peroxisome proliferator activated receptor signaling pathway [GO:0035360] (biological process) Sources: GOC:bf Relationships: is a type of GO:0035358; is_a positive regulation of intracellular signal transduction [GO:1902533]; positively regulates peroxisome proliferator activated receptor signaling pathway [GO:0035357] Also known as: positive regulation of PPAR signaling pathway, positive regulation of peroxisome proliferator activated receptor signalling pathway, positive regulation of peroxisome proliferator-activated receptor signaling pathway Definition: Any process that activates or increases the frequency, rate or extent of the peroxisome proliferator activated receptor signaling pathway.